{
  "gene_symbol": "LCE1B",
  "term_label": "Unknown cellular component",
  "gene": "UniProtKB:Q5T7P3",
  "gene_name": "Late cornified envelope protein 1B",
  "term_id": "UNKNOWN:0003"
}